{
  "gene": "UniProtKB:P09960",
  "term_label": "epoxide hydrolase activity",
  "gene_name": "Leukotriene A-4 hydrolase",
  "term_id": "GO:0004301",
  "gene_symbol": "LTA4H"
}